{
  "gene_name": "Small integral membrane protein 10-like protein 2A",
  "gene_symbol": "SMIM10L2A",
  "gene": "UniProtKB:P0DMW4",
  "term_label": "Unknown cellular component",
  "term_id": "UNKNOWN:0003"
}